internal mammary gland bud epithelial cell differentiation [GO:0060646] (biological process) Definition: The process in which a relatively unspecialized epithelial cell of the mammary placode becomes an internal epithelial cell of the mammary gland bud. Internal cells are small and of irregular shape. References: PMID:12558599 Sources: GOC:dph Relationships: is_a GO:0060643